{
  "gene_symbol": "CDC25A",
  "gene_name": "M-phase inducer phosphatase 1",
  "gene": "UniProtKB:P30304",
  "term_label": "positive regulation of G2/M transition of mitotic cell cycle",
  "term_id": "GO:0010971"
}